positive regulation of cellodextrin catabolic process [GO:2000929] (biological process) Definition: Any process that activates or increases the frequency, rate or extent of cellodextrin catabolic process. Also known as: positive regulation of cellodextrin catabolism Relationships: is a type of GO:0009896; is a type of positive regulation of macromolecule metabolic process [GO:0010604]; is_a GO:0045913; is a type of regulation of cellodextrin catabolic process [GO:2000927]; RO_0002213 cellodextrin catabolic process [GO:2000890] Sources: GOC:mengo_curators